{
  "gene_symbol": "TLX2",
  "gene": "UniProtKB:O43763",
  "term_id": "GO:0006357",
  "term_label": "regulation of transcription by RNA polymerase II",
  "gene_name": "T-cell leukemia homeobox protein 2"
}